cohesin loader activity [GO:0061775] (molecular function) Definition: Facilitating a conformational change to load a cohesin complex around sister chromatids. References: PMID:26687354 Sources: GOC:vw Relationships: is a type of catalytic activity, acting on DNA [GO:0140097] Also known as: cohesin loading activity